{
  "term_id": "UNKNOWN:0003",
  "term_label": "Unknown cellular component",
  "gene": "UniProtKB:Q70CQ4",
  "gene_name": "Ubiquitin carboxyl-terminal hydrolase 31",
  "gene_symbol": "USP31"
}